{
  "gene_name": "Tetraspanin-6",
  "term_id": "UNKNOWN:0001",
  "gene_symbol": "TSPAN6",
  "gene": "UniProtKB:O43657",
  "term_label": "Unknown molecular function"
}